{
  "gene_name": "Leucine-rich repeat-containing protein 14",
  "gene_symbol": "LRRC14",
  "gene": "UniProtKB:Q15048",
  "term_label": "negative regulation of toll-like receptor signaling pathway",
  "term_id": "GO:0034122"
}